3',3'-cyclic GMP-AMP binding [GO:0140703] (molecular function) Relationships: is a type of adenyl ribonucleotide binding [GO:0032559]; is a type of guanyl ribonucleotide binding [GO:0032561]; is_a anion binding [GO:0043168]; is a type of cyclic GMP-AMP binding [GO:0140702] Also known as: 3',3' cyclic-GMP-AMP binding, 3',3'-cGAMP binding, 3',3'-cGMP-AMP binding, 3',3'-cyclic GAMP binding Definition: Binding to 3',3' cyclic GMP-AMP (cGAMP) nucleotide, a cyclic purine dinucleotide that consists of AMP and GMP units cyclized via 3',5' and 3',5' linkages. References: PMID:30787435